dimethylpropiothetin dethiomethylase activity [GO:0047869] (molecular function) Sources: EC:4.4.1.3, RHEA:19965 Definition: Catalysis of the reaction: S,S-dimethyl-beta-propiothetin = acrylate + dimethyl sulfide + H+. Relationships: is a type of carbon-sulfur lyase activity [GO:0016846] Also known as: S,S-dimethyl-beta-propiothetin dimethyl-sulfide-lyase (acrylate-forming), S,S-dimethyl-beta-propiothetin dimethyl-sulfide-lyase activity, desulfhydrase activity